{
  "gene": "UniProtKB:Q99828",
  "term_id": "GO:0070886",
  "gene_symbol": "CIB1",
  "term_label": "positive regulation of calcineurin-NFAT signaling cascade",
  "gene_name": "Calcium and integrin-binding protein 1"
}